{
  "term_id": "GO:0004984",
  "gene": "UniProtKB:Q8NGP9",
  "gene_name": "Olfactory receptor 5AR1",
  "term_label": "olfactory receptor activity",
  "gene_symbol": "OR5AR1"
}